{
  "gene_name": "Beta-galactosidase-1-like protein 3",
  "term_id": "GO:0004565",
  "gene_symbol": "GLB1L3",
  "gene": "UniProtKB:Q8NCI6",
  "term_label": "beta-galactosidase activity"
}